{
  "gene_name": "Glycerate kinase",
  "term_label": "glycerate kinase activity",
  "gene": "UniProtKB:Q8IVS8",
  "gene_symbol": "GLYCTK",
  "term_id": "GO:0008887"
}